{
  "term_label": "Unknown cellular component",
  "gene": "UniProtKB:Q5VV16",
  "gene_symbol": "FOXD4L5",
  "term_id": "UNKNOWN:0003",
  "gene_name": "Forkhead box protein D4-like 5"
}